platelet activation [GO:0030168] (biological process) Definition: A series of progressive, overlapping events triggered by exposure of the platelets to subendothelial tissue. These events include shape change, adhesiveness, aggregation, and release reactions. When carried through to completion, these events lead to the formation of a stable hemostatic plug. Regulation: regulated by regulation of platelet activation [GO:0010543]; negatively regulated by negative regulation of platelet activation [GO:0010544]; positively regulated by positive regulation of platelet activation [GO:0010572] Relationships: is a type of cell activation [GO:0001775]; is part of blood coagulation [GO:0007596] References: PMID:27403440 Also known as: blood coagulation, platelet activation